{
  "gene_symbol": "TTC33",
  "term_label": "Unknown cellular component",
  "term_id": "UNKNOWN:0003",
  "gene_name": "Tetratricopeptide repeat protein 33",
  "gene": "UniProtKB:Q6PID6"
}